{
  "gene_symbol": "HTR4",
  "term_id": "GO:0004993",
  "term_label": "G protein-coupled serotonin receptor activity",
  "gene_name": "5-hydroxytryptamine receptor 4",
  "gene": "UniProtKB:Q13639"
}